negative regulation of fermentation [GO:1901003] (biological process) Sources: GOC:TermGenie Relationships: is a type of negative regulation of metabolic process [GO:0009892]; is_a regulation of fermentation [GO:0043465]; negatively regulates fermentation [GO:0006113] Subtypes: GO:1900516, negative regulation of glucose catabolic process to lactate via pyruvate [GO:1904024] Also known as: down regulation of fermentation, down-regulation of fermentation, downregulation of fermentation, inhibition of fermentation Definition: Any process that stops, prevents or reduces the frequency, rate or extent of fermentation.